{
  "term_id": "GO:0006805",
  "gene_symbol": "CYP2A7",
  "gene": "UniProtKB:P20853",
  "term_label": "xenobiotic metabolic process",
  "gene_name": "Cytochrome P450 2A7"
}